{
  "gene_symbol": "C1orf198",
  "term_id": "UNKNOWN:0002",
  "gene": "UniProtKB:Q9H425",
  "gene_name": "Uncharacterized protein C1orf198",
  "term_label": "Unknown biological process"
}